{
  "term_id": "GO:0141162",
  "gene_name": "High affinity cGMP-specific 3',5'-cyclic phosphodiesterase 9A",
  "gene_symbol": "PDE9A",
  "term_label": "negative regulation of cAMP/PKA signal transduction",
  "gene": "UniProtKB:O76083"
}